{
  "gene_name": "GDNF family receptor alpha-1",
  "gene": "UniProtKB:P56159",
  "term_label": "receptor complex",
  "term_id": "GO:0043235",
  "gene_symbol": "GFRA1"
}